mannogen catabolic process [GO:0106305] (biological process) Also known as: beta-1,2-mannan catabolic process, beta-1,2-mannan catabolism, mannogen breakdown, mannogen catabolism, mannogen degradation References: PMID:12902334, PMID:31513773, PMID:31662278 Relationships: is a type of GO:0000272 Definition: The chemical reactions and pathways resulting in the breakdown of mannogen, a mannose-containing polysaccharide that is a major energy reserve in Leishmania.